{
  "gene_name": "GDNF family receptor alpha-2",
  "term_label": "external side of plasma membrane",
  "term_id": "GO:0009897",
  "gene_symbol": "GFRA2",
  "gene": "UniProtKB:O00451"
}